{
  "gene": "UniProtKB:Q9BZ67",
  "term_id": "UNKNOWN:0001",
  "term_label": "Unknown molecular function",
  "gene_symbol": "FRMD8",
  "gene_name": "FERM domain-containing protein 8"
}